{
  "gene_name": "Thyroid hormone receptor alpha",
  "gene": "UniProtKB:P10827",
  "term_id": "GO:0000978",
  "term_label": "RNA polymerase II cis-regulatory region sequence-specific DNA binding",
  "gene_symbol": "THRA"
}